{
  "gene_name": "Agouti-signaling protein",
  "gene_symbol": "ASIP",
  "term_id": "GO:0031779",
  "gene": "UniProtKB:P42127",
  "term_label": "melanocortin receptor binding"
}